{
  "term_id": "UNKNOWN:0001",
  "gene": "UniProtKB:Q969S2",
  "gene_symbol": "NEIL2",
  "term_label": "Unknown molecular function",
  "gene_name": "Endonuclease 8-like 2"
}